{
  "term_label": "oxidoreductase activity, acting on paired donors, with incorporation or reduction of molecular oxygen, reduced flavin or flavoprotein as one donor, and incorporation of one atom of oxygen",
  "gene_symbol": "CYP2R1",
  "gene": "UniProtKB:Q6VVX0",
  "term_id": "GO:0016712",
  "gene_name": "Vitamin D 25-hydroxylase"
}